{
  "term_label": "Unknown biological process",
  "gene": "UniProtKB:A0A1B0GWG4",
  "gene_name": "Serine-rich and transmembrane domain-containing 2",
  "gene_symbol": "SERTM2",
  "term_id": "UNKNOWN:0002"
}